{
  "term_id": "UNKNOWN:0002",
  "gene_name": "Synaptojanin-2-binding protein",
  "gene_symbol": "SYNJ2BP",
  "term_label": "Unknown biological process",
  "gene": "UniProtKB:P57105"
}